{
  "gene_name": "Protein FAM76A",
  "gene_symbol": "FAM76A",
  "gene": "UniProtKB:Q8TAV0",
  "term_id": "GO:0016607",
  "term_label": "nuclear speck"
}